{
  "gene": "UniProtKB:Q96PL5",
  "gene_name": "Erythroid membrane-associated protein",
  "term_label": "regulation of cytokine production",
  "gene_symbol": "ERMAP",
  "term_id": "GO:0001817"
}